{
  "term_id": "GO:0032511",
  "gene": "UniProtKB:Q96CF2",
  "term_label": "late endosome to vacuole transport via multivesicular body sorting pathway",
  "gene_symbol": "CHMP4C",
  "gene_name": "Charged multivesicular body protein 4c"
}